determination of lung left/right asymmetry [GO:0140969] (BP) References: PMID:19944405, PMID:20007846, PMID:21131974 Sources: GOC:BHFL, GOC:rl Relationships: is a type of determination of left/right symmetry [GO:0007368]; is part of heart development [GO:0007507] Definition: Determination of the asymmetric location of the lungs with respect to the left and right halves of the organism.